{
  "gene": "UniProtKB:Q9BT81",
  "gene_symbol": "SOX7",
  "gene_name": "Transcription factor SOX-7",
  "term_id": "GO:0030154",
  "term_label": "cell differentiation"
}